{
  "gene": "UniProtKB:Q8NH19",
  "term_label": "plasma membrane",
  "gene_symbol": "OR10AG1",
  "gene_name": "Olfactory receptor 10AG1",
  "term_id": "GO:0005886"
}